{
  "term_id": "GO:0097352",
  "gene_name": "Gamma-aminobutyric acid receptor-associated protein",
  "term_label": "autophagosome maturation",
  "gene_symbol": "GABARAP",
  "gene": "UniProtKB:O95166"
}